positive regulation of telomerase catalytic core complex assembly [GO:1904884] (biological process) Relationships: is_a GO:0031334; is a type of regulation of telomerase catalytic core complex assembly [GO:1904882]; positively regulates GO:1904868 Definition: Any process that activates or increases the frequency, rate or extent of telomerase catalytic core complex assembly. References: PMID:26586433 Sources: GOC:BHF, GOC:BHF_telomere, GOC:TermGenie, GOC:rph, GO_REF:0000058 Also known as: positive regulation of telomerase catalytic core complex formation, up regulation of telomerase catalytic core complex assembly, up regulation of telomerase catalytic core complex formation, up-regulation of telomerase catalytic core complex assembly, up-regulation of telomerase catalytic core complex formation, upregulation of telomerase catalytic core complex assembly, upregulation of telomerase catalytic core complex formation, activation of telomerase catalytic core complex assembly, activation of telomerase catalytic core complex formation, activation of TERT-TERC complex assembly, activation of TERT-TERC complex formation, positive regulation of TERT-TERC complex assembly, positive regulation of TERT-TERC complex formation, up regulation of TERT-TERC complex assembly, up regulation of TERT-TERC complex formation, up-regulation of TERT-TERC complex assembly, up-regulation of TERT-TERC complex formation, upregulation of TERT-TERC complex assembly, upregulation of TERT-TERC complex formation